{
  "term_label": "ossification",
  "term_id": "GO:0001503",
  "gene_symbol": "TNFRSF11A",
  "gene": "UniProtKB:Q9Y6Q6",
  "gene_name": "Tumor necrosis factor receptor superfamily member 11A"
}